{
  "gene_symbol": "MUS81",
  "term_label": "mitotic intra-S DNA damage checkpoint signaling",
  "term_id": "GO:0031573",
  "gene_name": "Crossover junction endonuclease MUS81",
  "gene": "UniProtKB:Q96NY9"
}